glutathione metabolic process [GO:0006749] (biological process) Relationships: is a type of modified amino acid metabolic process [GO:0006575]; is a type of sulfur compound metabolic process [GO:0006790]; is a type of amide metabolic process [GO:0043603] Subtypes: glutathione biosynthetic process [GO:0006750], glutathione catabolic process [GO:0006751], ascorbate glutathione cycle [GO:0033355] Sources: ISBN:0198506732 Also known as: glutathione metabolism, oxidized glutathione reduction Definition: The chemical reactions and pathways involving glutathione, the tripeptide glutamylcysteinylglycine, which acts as a coenzyme for some enzymes and as an antioxidant in the protection of sulfhydryl groups in enzymes and other proteins; it has a specific role in the reduction of hydrogen peroxide (H2O2) and oxidized ascorbate, and it participates in the gamma-glutamyl cycle.